positive regulation of alcohol catabolic process [GO:1900421] (biological process) Sources: GOC:TermGenie Subtypes: positive regulation of 1,2-propanediol catabolic process [GO:0160161], positive regulation of ethanol catabolic process [GO:1900066] Definition: Any process that activates or increases the frequency, rate or extent of alcohol catabolic process within a cell. Also known as: up regulation of cellular alcohol catabolic process, up-regulation of cellular alcohol catabolic process, upregulation of cellular alcohol catabolic process, activation of cellular alcohol catabolic process Relationships: is a type of positive regulation of catabolic process [GO:0009896]; is a type of positive regulation of small molecule metabolic process [GO:0062013]; is a type of GO:1900419; positively regulates alcohol catabolic process [GO:0046164]